negative regulation of embryo sac central cell differentiation [GO:0045692] (BP) Relationships: is a type of negative regulation of cell differentiation [GO:0045596]; is a type of GO:0045691; is a type of negative regulation of multicellular organismal process [GO:0051241]; negatively regulates embryo sac central cell differentiation [GO:0009559] Sources: GOC:go_curators, GOC:mtg_plant Also known as: down regulation of female gametophyte central cell differentiation, down-regulation of female gametophyte central cell differentiation, downregulation of female gametophyte central cell differentiation, negative regulation of female gametophyte central cell differentiation, inhibition of female gametophyte central cell differentiation Definition: Any process that stops, prevents, or reduces the frequency, rate or extent of embryo sac central cell differentiation.